TRAPPIII protein complex [GO:1990072] (CC) References: PMID:20375281, PMID:22669257 Sources: GOC:bhm Definition: A complex that functions in anterograde transport at the Golgi and also regulates autophagy. In yeast it includes at least the following subunits: Bet3 (as homodimer), Bet5, Trs20, Trs23, Trs31, Trs33, Trs85. TRAPPIII may include further, as yet undescribed, proteins. Relationships: is a type of TRAPP complex [GO:0030008]; is part of Golgi apparatus [GO:0005794]